{
  "gene_name": "Coronin-7",
  "term_id": "GO:0051015",
  "gene_symbol": "CORO7",
  "gene": "UniProtKB:P57737",
  "term_label": "actin filament binding"
}